cholesterol ester hydrolysis involved in cholesterol transport [GO:0090122] (biological process) Definition: The cholesterol metabolic process in which cholesterol esters are hydrolyzed into free fatty acids and cholesterol in the lysosome that contributes to intracellular cholesterol transport. Sources: GOC:ascb_2009, GOC:dph, GOC:tb Relationships: is a type of cholesterol metabolic process [GO:0008203]; is part of vesicle-mediated cholesterol transport [GO:0090119]